{
  "term_label": "peroxisome",
  "gene_name": "Fatty acyl-CoA reductase 1",
  "gene": "UniProtKB:Q8WVX9",
  "gene_symbol": "FAR1",
  "term_id": "GO:0005777"
}